{
  "gene_name": "Docking protein 1",
  "gene_symbol": "DOK1",
  "gene": "UniProtKB:Q99704",
  "term_label": "signaling adaptor activity",
  "term_id": "GO:0035591"
}